{
  "gene_symbol": "ZMPSTE24",
  "term_label": "endoplasmic reticulum membrane",
  "gene_name": "CAAX prenyl protease 1 homolog",
  "gene": "UniProtKB:O75844",
  "term_id": "GO:0005789"
}